postsynapse assembly [GO:0099068] (biological process) Definition: The aggregation, arrangement and bonding together of a set of components to form a postsynapse. Sources: GOC:bf, GOC:dos, GOCL:PARL Also known as: postsynapse biogenesis Relationships: is a type of cellular component assembly [GO:0022607]; is a type of postsynapse organization [GO:0099173]; is part of synapse assembly [GO:0007416] Regulation: regulated by regulation of postsynapse assembly [GO:0150052]